leukocyte activation involved in immune response [GO:0002366] (biological process) Also known as: immune cell activation during immune response, leucocyte activation during immune response, leukocyte activation during immune response Definition: A change in morphology and behavior of a leukocyte resulting from exposure to a specific antigen, mitogen, cytokine, cellular ligand, or soluble factor, leading to the initiation or perpetuation of an immune response. Sources: GOC:add, ISBN:0781735149 Subtypes: plasmacytoid dendritic cell activation involved in immune response [GO:0002271], myeloid cell activation involved in immune response [GO:0002275], GO:0002276, GO:0002281, GO:0002285 Relationships: is_a cell activation involved in immune response [GO:0002263]; is a type of leukocyte activation [GO:0045321]